{
  "gene": "UniProtKB:Q15650",
  "gene_name": "Activating signal cointegrator 1",
  "gene_symbol": "TRIP4",
  "term_id": "GO:0005634",
  "term_label": "nucleus"
}